{
  "gene_name": "Protocadherin Fat 3",
  "term_label": "cell-cell adhesion mediated by cadherin",
  "gene_symbol": "FAT3",
  "gene": "UniProtKB:Q8TDW7",
  "term_id": "GO:0044331"
}